{
  "gene_name": "YTH domain-containing family protein 3",
  "term_id": "GO:0005737",
  "gene": "UniProtKB:Q7Z739",
  "term_label": "cytoplasm",
  "gene_symbol": "YTHDF3"
}